{
  "gene": "UniProtKB:Q9Y4Z2",
  "gene_name": "Neurogenin-3",
  "gene_symbol": "NEUROG3",
  "term_id": "GO:0005634",
  "term_label": "nucleus"
}